positive regulation of central B cell anergy [GO:0002916] (biological process) Relationships: is a type of GO:0002672; is a type of GO:0002897; is a type of GO:0002914; is a type of positive regulation of B cell differentiation [GO:0045579]; positively regulates GO:0002341 Also known as: up regulation of central B cell anergy, up-regulation of central B cell anergy, upregulation of central B cell anergy, activation of central B cell anergy, stimulation of central B cell anergy Definition: Any process that activates or increases the frequency, rate, or extent of central B cell anergy. Sources: GOC:add